{
  "gene_name": "Large ribosomal subunit protein eL38",
  "gene_symbol": "RPL38",
  "term_id": "GO:0022625",
  "term_label": "cytosolic large ribosomal subunit",
  "gene": "UniProtKB:P63173"
}